 [go#goslim:synapse] Note: synapse GO slim